1-aminocyclopropane-1-carboxylate catabolic process [GO:0042217] (biological process) Sources: GOC:go_curators Relationships: is a type of 1-aminocyclopropane-1-carboxylate metabolic process [GO:0018871]; is a type of GO:0170044; is a type of alpha-amino acid catabolic process [GO:1901606] Also known as: 1-aminocyclopropane-1-carboxylate breakdown, 1-aminocyclopropane-1-carboxylate catabolism, 1-aminocyclopropane-1-carboxylate degradation Definition: The chemical reactions and pathways resulting in the breakdown of 1-aminocyclopropane-1-carboxylate, a natural product found in plant tissues. It is a key intermediate in the biosynthesis of ethylene (ethene), a fruit-ripening hormone in plants.